{
  "term_id": "UNKNOWN:0001",
  "gene_symbol": "C22orf42",
  "gene": "UniProtKB:Q6IC83",
  "term_label": "Unknown molecular function",
  "gene_name": "Uncharacterized protein C22orf42"
}